{
  "term_id": "GO:0015030",
  "gene": "UniProtKB:Q16637",
  "gene_name": "Survival motor neuron protein",
  "term_label": "Cajal body",
  "gene_symbol": "SMN2"
}